positive regulation of sphingolipid biosynthetic process [GO:0090154] (biological process) Sources: GOC:ascb_2009, GOC:dph, GOC:tb Relationships: is a type of GO:0046889; is a type of regulation of sphingolipid biosynthetic process [GO:0090153]; positively regulates GO:0030148 Definition: Any process that increases the rate, frequency or extent of sphingolipid biosynthesis. Sphingolipid biosynthesis is the chemical reactions and pathways resulting in the formation of sphingolipids, any of a class of lipids containing the long-chain amine diol sphingosine or a closely related base (a sphingoid). Subtypes: positive regulation of ceramide biosynthetic process [GO:2000304]